{
  "gene_name": "Oligodendrocyte transcription factor 2",
  "term_label": "positive regulation of transcription by RNA polymerase II",
  "gene_symbol": "OLIG2",
  "gene": "UniProtKB:Q13516",
  "term_id": "GO:0045944"
}